{
  "term_label": "regulation of mRNA processing",
  "gene_symbol": "SRPK1",
  "gene_name": "SRSF protein kinase 1",
  "term_id": "GO:0050684",
  "gene": "UniProtKB:Q96SB4"
}